{
  "gene_symbol": "TIMM23B",
  "term_label": "protein import into mitochondrial matrix",
  "term_id": "GO:0030150",
  "gene_name": "Mitochondrial import inner membrane translocase subunit Tim23B",
  "gene": "UniProtKB:Q5SRD1"
}